{
  "gene_symbol": "TIAM1",
  "gene": "UniProtKB:Q13009",
  "term_id": "GO:0050772",
  "term_label": "positive regulation of axonogenesis",
  "gene_name": "Rho guanine nucleotide exchange factor TIAM1"
}